glyceraldehyde-3-phosphate dehydrogenase [NAD(P)+] (non-phosphorylating) activity [GO:0120533] (molecular function) Relationships: is a type of oxidoreductase activity, acting on the aldehyde or oxo group of donors, NAD or NADP as acceptor [GO:0016620] Also known as: GAPN activity, non-phosphorylating glyceraldehyde-3-phosphate dehydrogenase activity Sources: EC:1.2.1.90 Definition: Catalysis of the reaction: D-glyceraldehyde 3-phosphate + NAD(P)+ + H2O = (2R)-3-phosphoglycerate + NAD(P)H + 2 H+. Subtypes: glyceraldehyde-3-phosphate dehydrogenase (NADP+) (non-phosphorylating) activity [GO:0008886], glyceraldehyde-3-phosphate dehydrogenase (NAD+) (non-phosphorylating) activity [GO:0043878]